{
  "term_label": "vacuolar proton-transporting V-type ATPase complex",
  "term_id": "GO:0016471",
  "gene": "UniProtKB:P61421",
  "gene_symbol": "ATP6V0D1",
  "gene_name": "V-type proton ATPase subunit d 1"
}